sensory perception of salty taste [GO:0050914] (biological process) Definition: The series of events required to receive a salty taste stimulus, convert it to a molecular signal, and recognize and characterize the signal. This is a neurological process. Relationships: is a type of sensory perception of taste [GO:0050909] Also known as: salty taste perception Sources: GOC:ai